{
  "gene_name": "Whirlin",
  "term_label": "plasma membrane",
  "gene_symbol": "WHRN",
  "gene": "UniProtKB:Q9P202",
  "term_id": "GO:0005886"
}